{
  "gene_symbol": "SPICE1",
  "gene": "UniProtKB:Q8N0Z3",
  "gene_name": "Spindle and centriole-associated protein 1",
  "term_label": "centriole",
  "term_id": "GO:0005814"
}